negative regulation of cellular component organization [GO:0051129] (BP) Relationships: is_a negative regulation of cellular process [GO:0048523]; is a type of regulation of cellular component organization [GO:0051128]; negatively regulates cellular component organization [GO:0016043] Subtypes: negative regulation of organelle organization [GO:0010639], negative regulation of very-low-density lipoprotein particle remodeling [GO:0010903], GO:0031333, negative regulation of cell projection organization [GO:0031345], negative regulation of syncytium formation by plasma membrane fusion [GO:0034242], negative regulation of plasma lipoprotein oxidation [GO:0034445], negative regulation of fusion of sperm to egg plasma membrane [GO:0043013], negative regulation of protein-containing complex disassembly [GO:0043242], negative regulation of integrin biosynthetic process [GO:0045720], negative regulation of endocytosis [GO:0045806], negative regulation of synapse structural plasticity [GO:0051826], GO:0061093, negative regulation of erythrocyte enucleation [GO:0061932], negative regulation of inclusion body assembly [GO:0090084], negative regulation of cell-substrate junction organization [GO:0150118], GO:1900105, negative regulation of terminal button organization [GO:1901613], negative regulation of synaptic vesicle membrane organization [GO:1901633], GO:1901889, negative regulation of cell septum assembly [GO:1901892], negative regulation of capsule organization [GO:1901914], GO:1902904, GO:1903054, negative regulation of vitellogenesis [GO:1903187], negative regulation of iron-sulfur cluster assembly [GO:1903330], negative regulation of adherens junction organization [GO:1903392], negative regulation of membrane tubulation [GO:1903526], negative regulation of plasma membrane raft polarization [GO:1903907], negative regulation of fusion of virus membrane with host plasma membrane [GO:1903914], negative regulation of t-circle formation [GO:1904430], negative regulation of tight junction disassembly [GO:1905074], GO:1905154, negative regulation of chromatin organization [GO:1905268], negative regulation of mitotic nuclear envelope disassembly [GO:1905558], GO:1905685, GO:1905809, GO:2000333, negative regulation of barbed-end actin filament capping [GO:2000813] Definition: Any process that stops, prevents, or reduces the frequency, rate or extent of a process involved in the formation, arrangement of constituent parts, or disassembly of cell structures, including the plasma membrane and any external encapsulating structures such as the cell wall and cell envelope. Sources: GOC:ai Also known as: down regulation of cell organization, down-regulation of cell organization, downregulation of cell organization, inhibition of cell organization, negative regulation of cell organisation, negative regulation of cellular component organization and biogenesis